guanyl-nucleotide exchange factor activity [GO:0005085] (molecular function) Relationships: is a type of GTPase regulator activity [GO:0030695]; negatively regulates GDP binding [GO:0019003]; RO_0002213 GTP binding [GO:0005525] Also known as: GDP-dissociation stimulator activity, GDS, GEF, Rho guanine nucleotide exchange factor, RhoGEF, guanyl-nucleotide release factor activity, guanyl-nucleotide releasing factor, ARF guanyl-nucleotide exchange factor activity, GNRP, Rab guanyl-nucleotide exchange factor activity, Rac guanyl-nucleotide exchange factor activity, Ral guanyl-nucleotide exchange factor activity, Ran guanyl-nucleotide exchange factor activity, Rap guanyl-nucleotide exchange factor activity, Ras guanyl-nucleotide exchange factor activity, Rho guanyl-nucleotide exchange factor activity, Sar guanyl-nucleotide exchange factor activity, cAMP-dependent guanyl-nucleotide exchange factor activity Definition: Stimulates the exchange of GDP to GTP on a signaling GTPase, changing its conformation to its active form. Guanine nucleotide exchange factors (GEFs) act by stimulating the release of guanosine diphosphate (GDP) to allow binding of guanosine triphosphate (GTP), which is more abundant in the cell under normal cellular physiological conditions. Regulation: negatively regulated by GO:1905098 References: PMID:23303910, PMID:27218782 Sources: GOC:kd, GOC:mah